{
  "gene_name": "Ras-related GTP-binding protein D",
  "gene": "UniProtKB:Q9NQL2",
  "gene_symbol": "RRAGD",
  "term_label": "positive regulation of TORC1 signaling",
  "term_id": "GO:1904263"
}